forebrain development [GO:0030900] (biological process) Relationships: is a type of GO:0048856; is part of brain development [GO:0007420] Also known as: prosencephalon development Definition: The process whose specific outcome is the progression of the forebrain over time, from its formation to the mature structure. The forebrain is the anterior of the three primary divisions of the developing chordate brain or the corresponding part of the adult brain (in vertebrates, includes especially the cerebral hemispheres, the thalamus, and the hypothalamus and especially in higher vertebrates is the main control center for sensory and associative information processing, visceral functions, and voluntary motor functions). References: PMID:4975589, PMID:4992177